{
  "term_id": "UNKNOWN:0003",
  "gene": "UniProtKB:Q5TBE3",
  "gene_name": "Uncharacterized protein C9orf153",
  "gene_symbol": "C9orf153",
  "term_label": "Unknown cellular component"
}